{
  "gene": "UniProtKB:Q9H6R4",
  "term_id": "GO:0032040",
  "gene_symbol": "NOL6",
  "gene_name": "Nucleolar protein 6",
  "term_label": "small-subunit processome"
}